{
  "gene_symbol": "ZNF614",
  "gene_name": "Zinc finger protein 614",
  "term_label": "regulation of transcription by RNA polymerase II",
  "gene": "UniProtKB:Q8N883",
  "term_id": "GO:0006357"
}